{
  "gene_name": "Zinc finger protein 124",
  "gene": "UniProtKB:Q15973",
  "term_label": "RNA polymerase II transcription regulatory region sequence-specific DNA binding",
  "gene_symbol": "ZNF124",
  "term_id": "GO:0000977"
}